{
  "gene_symbol": "ADGRB1",
  "term_label": "engulfment of apoptotic cell",
  "term_id": "GO:0043652",
  "gene": "UniProtKB:O14514",
  "gene_name": "Adhesion G protein-coupled receptor B1"
}